acidocalcisome membrane [GO:0033102] (cellular component) Definition: The lipid bilayer surrounding an acidocalcisome. Relationships: is a type of bounding membrane of organelle [GO:0098588]; is part of acidocalcisome [GO:0020022] References: PMID:11378195 Sources: GOC:ecd